{
  "gene_name": "Chloride channel protein 2",
  "term_id": "GO:0005247",
  "term_label": "voltage-gated chloride channel activity",
  "gene": "UniProtKB:P51788",
  "gene_symbol": "CLCN2"
}